{
  "term_label": "Unknown biological process",
  "gene": "UniProtKB:P07910",
  "gene_symbol": "HNRNPC",
  "term_id": "UNKNOWN:0002",
  "gene_name": "Heterogeneous nuclear ribonucleoproteins C1_C2"
}